deadenylation-dependent decapping of nuclear-transcribed mRNA [GO:0000290] (biological process) Regulation: regulated by GO:0106288; negatively regulated by negative regulation of deadenylation-dependent decapping of nuclear-transcribed mRNA [GO:0106289] Sources: GOC:krc Definition: Cleavage of the 5'-cap of a nuclear mRNA triggered by shortening of the poly(A) tail to below a minimum functional length. Relationships: is a type of nuclear-transcribed mRNA catabolic process [GO:0000956]; is_a mRNA methylguanosine-cap decapping [GO:0110156]; is part of nuclear-transcribed mRNA catabolic process, deadenylation-dependent decay [GO:0000288] Also known as: deadenylation-dependent decapping of nuclear mRNA, deadenylylation-dependent decapping